{
  "gene_name": "Kinesin-like protein KIF14",
  "gene": "UniProtKB:Q15058",
  "term_label": "cytoplasm",
  "term_id": "GO:0005737",
  "gene_symbol": "KIF14"
}